negative regulation of endothelial cell migration [GO:0010596] (biological process) Sources: GOC:BHF, GOC:dph, GOC:tb Subtypes: negative regulation of blood vessel endothelial cell migration [GO:0043537], GO:2001027 Relationships: is a type of GO:0010594; is a type of negative regulation of cell migration [GO:0030336]; negatively regulates GO:0043542 Definition: Any process that decreases the rate, frequency, or extent of the orderly movement of an endothelial cell into the extracellular matrix to form an endothelium.